{
  "term_id": "GO:0006357",
  "gene": "UniProtKB:Q6ZN06",
  "gene_symbol": "ZNF813",
  "gene_name": "Zinc finger protein 813",
  "term_label": "regulation of transcription by RNA polymerase II"
}